positive regulation of calcium-mediated signaling involved in cellular response to calcium ion [GO:1901197] (biological process) Sources: GOC:TermGenie Relationships: is a type of positive regulation of calcium-mediated signaling [GO:0050850]; is part of cellular response to calcium ion [GO:0071277] Definition: Any positive regulation of calcium-mediated signaling that is involved in cellular response to calcium ion. Also known as: positive regulation of calcium-mediated signaling involved in cellular response to Ca2+ ion, positive regulation of calcium-mediated signalling involved in cellular response to Ca2+ ion, positive regulation of calcium-mediated signalling involved in cellular response to calcium ion, up regulation of calcium-mediated signaling involved in cellular response to Ca2+ ion, up regulation of calcium-mediated signaling involved in cellular response to calcium ion, up-regulation of calcium-mediated signaling involved in cellular response to Ca2+ ion, up-regulation of calcium-mediated signaling involved in response to calcium ion, upregulation of calcium-mediated signaling involved in cellular response to Ca2+ ion, upregulation of calcium-mediated signaling involved in cellular response to calcium ion, activation of calcium-mediated signaling involved in cellular response to Ca2+ ion, activation of calcium-mediated signaling involved in cellular response to calcium ion, stimulation of calcium-mediated signaling involved in cellular response to Ca2+ ion, stimulation of calcium-mediated signaling involved in cellular response to calcium ion